{
  "gene": "UniProtKB:Q9Y6X3",
  "term_label": "maintenance of mitotic sister chromatid cohesion",
  "gene_symbol": "MAU2",
  "gene_name": "MAU2 chromatid cohesion factor homolog",
  "term_id": "GO:0034088"
}